{
  "term_label": "cell-cell adhesion mediated by cadherin",
  "gene_symbol": "CDH22",
  "gene_name": "Cadherin-22",
  "gene": "UniProtKB:Q9UJ99",
  "term_id": "GO:0044331"
}